{
  "term_label": "external side of plasma membrane",
  "gene": "UniProtKB:Q9BZM5",
  "gene_name": "UL16-binding protein 2",
  "gene_symbol": "ULBP2",
  "term_id": "GO:0009897"
}